{
  "term_label": "phospholipase A1 activity",
  "gene_name": "Pancreatic triacylglycerol lipase",
  "gene_symbol": "PNLIP",
  "term_id": "GO:0008970",
  "gene": "UniProtKB:P16233"
}